{
  "gene_symbol": "SLURP2",
  "term_label": "acetylcholine receptor signaling pathway",
  "gene_name": "Secreted Ly-6_uPAR domain-containing protein 2",
  "gene": "UniProtKB:P0DP57",
  "term_id": "GO:0095500"
}